response to BMP [GO:0071772] (biological process) Sources: GOC:mah, GOC:yaf Definition: Any process that results in a change in state or activity of a cell or an organism (in terms of movement, secretion, enzyme production, gene expression, etc.) as a result of a bone morphogenetic protein (BMP) stimulus. Relationships: is_a response to growth factor [GO:0070848] Subtypes: cellular response to BMP stimulus [GO:0071773] Also known as: response to BMP stimulus, response to bone morphogenetic protein stimulus